{
  "gene_symbol": "SYTL5",
  "gene": "UniProtKB:Q8TDW5",
  "gene_name": "Synaptotagmin-like protein 5",
  "term_id": "GO:0005886",
  "term_label": "plasma membrane"
}